response to Gentian violet [GO:0072728] (biological process) Sources: GOC:mah Subtypes: cellular response to Gentian violet [GO:0072729] Relationships: is a type of GO:0042221 Definition: Any process that results in a change in state or activity of a cell or an organism (in terms of movement, secretion, enzyme production, gene expression, etc.) as a result of a Gentian violet stimulus. Also known as: response to crystal violet, response to {4-[Bis-(4-dimethylamino-phenyl)-methylene]-cyclohexa-2,5-dienylidene}-dimethyl-ammonium chloride